{
  "term_label": "RNA polymerase II cis-regulatory region sequence-specific DNA binding",
  "gene_symbol": "ATF1",
  "gene": "UniProtKB:P18846",
  "term_id": "GO:0000978",
  "gene_name": "Cyclic AMP-dependent transcription factor ATF-1"
}